{
  "gene_name": "Putative small nuclear ribonucleoprotein G-like protein 15",
  "term_id": "GO:0034719",
  "gene_symbol": "SNRPGP15",
  "gene": "UniProtKB:A8MWD9",
  "term_label": "SMN-Sm protein complex"
}